{
  "gene_symbol": "SLC43A1",
  "term_label": "L-amino acid transmembrane transporter activity",
  "gene": "UniProtKB:O75387",
  "term_id": "GO:0015179",
  "gene_name": "Large neutral amino acids transporter small subunit 3"
}